{
  "gene_symbol": "CTNND1",
  "gene": "UniProtKB:O60716",
  "term_label": "adherens junction",
  "gene_name": "Catenin delta-1",
  "term_id": "GO:0005912"
}